methionyl-tRNA formyltransferase activity [GO:0004479] (molecular function) Also known as: 10-formyltetrahydrofolate:L-methionyl-tRNA N-formyltransferase activity, N(10)-formyltetrahydrofolic-methionyl-transfer ribonucleic transformylase activity, N-terminal peptidyl-methionine N-formylation, N10-formyltetrahydrofolic-methionyl-transfer ribonucleic transformylase activity, conversion of met-tRNAf to fmet-tRNA, conversion of mitochondrial met-tRNAf to fmet-tRNA, formylmethionyl-transfer ribonucleic synthetase activity, methionyl ribonucleic formyltransferase activity, methionyl-tRNA Met formyltransferase activity, methionyl-tRNA transformylase activity, methionyl-transfer RNA transformylase activity, methionyl-transfer ribonucleate methyltransferase activity, methionyl-transfer ribonucleic transformylase activity, mitochondrial N-terminal peptidyl-methionine N-formylation Relationships: is a type of hydroxymethyl-, formyl- and related transferase activity [GO:0016742]; is a type of catalytic activity, acting on a tRNA [GO:0140101]; is part of translational initiation [GO:0006413]; is part of conversion of methionyl-tRNA to N-formyl-methionyl-tRNA [GO:0071951] Sources: EC:2.1.2.9 Definition: Catalysis of the reaction: 10-formyltetrahydrofolate + L-methionyl-tRNA + H2O = tetrahydrofolate + N-formylmethionyl-tRNA.